maintenance of dense core granule location [GO:0032257] (biological process) Also known as: maintenance of dense core vesicle location, maintenance of dense core granule localization Sources: GOC:dph, GOC:mah, GOC:tb Relationships: is a type of GO:0032255; is part of dense core granule localization [GO:0032253] Definition: Any process in which a dense core granule is maintained in a specific location within a cell and prevented from moving elsewhere.